{
  "gene": "UniProtKB:Q5VZ19",
  "term_id": "GO:0005739",
  "gene_symbol": "TDRD10",
  "gene_name": "Tudor domain-containing protein 10",
  "term_label": "mitochondrion"
}